{
  "term_label": "homophilic cell-cell adhesion",
  "term_id": "GO:0007156",
  "gene": "UniProtKB:P32004",
  "gene_name": "Neural cell adhesion molecule L1",
  "gene_symbol": "L1CAM"
}